{
  "gene_name": "Cyclic nucleotide-gated cation channel beta-1",
  "term_label": "intracellularly cAMP-activated cation channel activity",
  "gene": "UniProtKB:Q14028",
  "term_id": "GO:0005222",
  "gene_symbol": "CNGB1"
}